primary alcohol catabolic process [GO:0034310] (biological process) Also known as: monohydric alcohol catabolic process, primary alcohol breakdown, primary alcohol catabolism, primary alcohol degradation Relationships: is a type of primary alcohol metabolic process [GO:0034308]; is a type of alcohol catabolic process [GO:0046164] Definition: The chemical reactions and pathways resulting in the breakdown of primary alcohols. A primary alcohol is any alcohol in which a hydroxy group, -OH, is attached to a saturated carbon atom which has either three hydrogen atoms attached to it or only one other carbon atom and two hydrogen atoms attached to it. Subtypes: ethanol catabolic process [GO:0006068], thiamine catabolic process [GO:0009230], farnesol catabolic process [GO:0016488], aldosterone catabolic process [GO:0032343], GO:0042859, methanol catabolic process [GO:0046170], GO:0046172, GO:0046296, GO:0046336, (+)-lariciresinol catabolic process [GO:1902131], GO:1903447 Sources: GOC:mah